{
  "term_id": "GO:0030182",
  "gene_symbol": "WNT4",
  "term_label": "neuron differentiation",
  "gene_name": "Protein Wnt-4",
  "gene": "UniProtKB:P56705"
}